{
  "term_label": "Unknown cellular component",
  "gene_symbol": "FAM168B",
  "gene": "UniProtKB:A1KXE4",
  "term_id": "UNKNOWN:0003",
  "gene_name": "Myelin-associated neurite-outgrowth inhibitor"
}